phosphonopyruvate decarboxylase activity [GO:0033980] (molecular function) Definition: Catalysis of the reaction: 3-phosphonopyruvate + 2 H+ = CO2 + phosphonoacetaldehyde. Relationships: is a type of carboxy-lyase activity [GO:0016831] Also known as: 3-phosphonopyruvate carboxy-lyase (2-phosphonoacetaldehyde-forming) activity, 3-phosphonopyruvate carboxy-lyase activity Sources: EC:4.1.1.82, RHEA:20768